aminoacyl-tRNA deacylase activity [GO:0002161] (MF) Relationships: is a type of carboxylic ester hydrolase activity [GO:0052689]; is_a catalytic activity, acting on a tRNA [GO:0140101]; is_a deacylase activity [GO:0160215]; BFO_0000050 aminoacyl-tRNA metabolism involved in translational fidelity [GO:0106074] Subtypes: Ser-tRNA(Ala) deacylase activity [GO:0002196], Ala-tRNA(Pro) deacylase activity [GO:0043906], Cys-tRNA(Pro) deacylase activity [GO:0043907], GO:0051499, GO:0106026, GO:0106105 Definition: The hydrolysis of an incorrectly aminoacylated tRNA. References: PMID:14663147, PMID:16087889 Sources: GOC:hjd Also known as: aminoacyl-tRNA editing activity, amino acid proofreading activity, aminoacyl-tRNA hydrolysis activity